{
  "gene_symbol": "AHI1-DT",
  "term_id": "UNKNOWN:0002",
  "gene": "UniProtKB:P0C7V0",
  "term_label": "Unknown biological process",
  "gene_name": "Putative uncharacterized protein encoded by LINC00271"
}